structural constituent of synapse [GO:0098918] (molecular function) Sources: GOC:dos Subtypes: structural constituent of presynaptic active zone [GO:0098882], structural constituent of presynapse [GO:0099181], structural constituent of postsynapse [GO:0099186] Relationships: is a type of structural molecule activity [GO:0005198]; is part of synapse organization [GO:0050808]; occurs in synapse [GO:0045202] Definition: The action of a molecule that contributes to the structural integrity of a synapse.